{
  "gene": "UniProtKB:Q15528",
  "gene_name": "Mediator of RNA polymerase II transcription subunit 22",
  "gene_symbol": "MED22",
  "term_label": "mediator complex",
  "term_id": "GO:0016592"
}